{
  "term_label": "endoplasmic reticulum membrane",
  "term_id": "GO:0005789",
  "gene_name": "Long-chain fatty acid transport protein 2",
  "gene_symbol": "SLC27A2",
  "gene": "UniProtKB:O14975"
}